{
  "term_label": "Unknown molecular function",
  "gene": "UniProtKB:A0A1W2PPE3",
  "gene_symbol": "C1orf202",
  "term_id": "UNKNOWN:0001",
  "gene_name": "Uncharacterized protein C1orf202"
}